translation at presynapse [GO:0140236] (biological process) Note: Note that this term was created for the SynGO project, and will be obsoleted when the SynGO annotations are made in Noctua. References: PMID:27321671 Definition: Translation that occurs at the presynapse. Subtypes: translation at presynapse, modulating chemical synaptic transmission [GO:0140237] Relationships: is a type of translation at synapse [GO:0140241]; occurs in presynapse [GO:0098793]